{
  "gene_name": "cAMP-responsive element-binding protein-like 2",
  "gene_symbol": "CREBL2",
  "term_label": "regulation of DNA-templated transcription",
  "gene": "UniProtKB:O60519",
  "term_id": "GO:0006355"
}